{
  "term_id": "GO:0005024",
  "gene_symbol": "AMHR2",
  "gene_name": "Anti-Muellerian hormone type-2 receptor",
  "term_label": "transforming growth factor beta receptor activity",
  "gene": "UniProtKB:Q16671"
}